{
  "gene_symbol": "GABPA",
  "term_label": "DNA-binding transcription factor activity, RNA polymerase II-specific",
  "gene_name": "GA-binding protein alpha chain",
  "gene": "UniProtKB:Q06546",
  "term_id": "GO:0000981"
}